{
  "gene_name": "Putative protein RNF216-like",
  "gene_symbol": "RNF216P1",
  "term_label": "Unknown cellular component",
  "gene": "UniProtKB:Q6NUR6",
  "term_id": "UNKNOWN:0003"
}